viral budding from Golgi membrane [GO:0046760] (biological process) Also known as: Golgi membrane viral budding, virus budding from Golgi membrane, Golgi membrane viral budding during viral capsid envelopment, viral budding from Golgi membrane by viral capsid envelopment, viral budding from Golgi membrane during viral capsid envelopment, virus budding from Golgi membrane by viral capsid envelopment, virus budding from Golgi membrane during viral capsid envelopment Relationships: is a type of viral budding [GO:0046755] Sources: GOC:bf, ISBN:0072370319, VZ:1947 Definition: A viral budding that starts with formation of a membrane curvature in the host Golgi membrane.